{
  "gene": "UniProtKB:Q6DN03",
  "term_label": "extracellular space",
  "term_id": "GO:0005615",
  "gene_name": "Putative histone H2B type 2-C",
  "gene_symbol": "H2BC20P"
}